{
  "gene": "UniProtKB:P13674",
  "gene_symbol": "P4HA1",
  "term_label": "collagen fibril organization",
  "gene_name": "Prolyl 4-hydroxylase subunit alpha-1",
  "term_id": "GO:0030199"
}